motor neuron apoptotic process [GO:0097049] (biological process) Also known as: motoneuron apoptosis, motor neuron apoptosis Regulation: regulated by regulation of motor neuron apoptotic process [GO:2000671]; RO_0002212 by negative regulation of motor neuron apoptotic process [GO:2000672]; positively regulated by positive regulation of motor neuron apoptotic process [GO:2000673] References: PMID:14523086 Sources: CL:0000100, GOC:BHF, GOC:mtg_apoptosis Relationships: is a type of neuron apoptotic process [GO:0051402] Definition: Any apoptotic process in a motor neuron, an efferent neuron that passes from the central nervous system or a ganglion toward or to a muscle and conducts an impulse that causes movement.